demethylase activity [GO:0032451] (molecular function) Definition: Catalysis of the removal of a methyl group from a substrate. Sources: GOC:mah Relationships: is a type of catalytic activity [GO:0003824] Subtypes: sterol 14-demethylase activity [GO:0008398], vanillate monooxygenase activity [GO:0018489], GO:0035514, oxidative RNA demethylase activity [GO:0035515], GO:0098608, GO:0140457